{
  "gene": "UniProtKB:Q6UB28",
  "term_label": "Unknown biological process",
  "gene_symbol": "METAP1D",
  "gene_name": "Methionine aminopeptidase 1D, mitochondrial",
  "term_id": "UNKNOWN:0002"
}